{
  "gene_symbol": "TSEN15",
  "gene": "UniProtKB:Q8WW01",
  "term_id": "UNKNOWN:0001",
  "term_label": "Unknown molecular function",
  "gene_name": "tRNA-splicing endonuclease subunit Sen15"
}